{
  "gene_symbol": "PCK2",
  "gene_name": "Phosphoenolpyruvate carboxykinase [GTP], mitochondrial",
  "term_label": "cellular response to dexamethasone stimulus",
  "gene": "UniProtKB:Q16822",
  "term_id": "GO:0071549"
}